{
  "gene": "UniProtKB:Q9BZG1",
  "gene_symbol": "RAB34",
  "term_label": "GTPase activity",
  "term_id": "GO:0003924",
  "gene_name": "Ras-related protein Rab-34"
}